sequence-specific mRNA binding [GO:1990825] (molecular function) Definition: Binding to messenger RNA (mRNA) of a specific nucleotide composition or a specific sequence motif. References: PMID:11886857 Relationships: is a type of mRNA binding [GO:0003729] Subtypes: mRNA base-pairing post-transcriptional repressor activity [GO:1903231]